negative regulation of cell cycle [GO:0045786] (biological process) Definition: Any process that stops, prevents or reduces the rate or extent of progression through the cell cycle. Also known as: down regulation of progression through cell cycle, down-regulation of progression through cell cycle, downregulation of progression through cell cycle, negative regulation of cell cycle progression, negative regulation of progression through cell cycle, inhibition of progression through cell cycle Subtypes: negative regulation of cell cycle process [GO:0010948], negative regulation of cyclin-dependent protein serine/threonine kinase activity [GO:0045736], GO:0045930, GO:0051447 Relationships: is a type of negative regulation of cellular process [GO:0048523]; is a type of regulation of cell cycle [GO:0051726]; negatively regulates GO:0007049 Sources: GOC:dph, GOC:go_curators, GOC:tb